fibroblast growth factor receptor signaling pathway involved in spinal cord anterior/posterior pattern formation [GO:0021907] (biological process) Also known as: fibroblast growth factor receptor signalling pathway in spinal cord anterior-posterior patterning Relationships: is a type of GO:0008543; is part of spinal cord anterior/posterior patterning [GO:0021512] References: PMID:11262869 Sources: GOC:cls, GOC:dgh, GOC:dph, GOC:jid, GO_REF:0000021 Definition: The series of molecular signals generated as a consequence of a fibroblast growth factor receptor binding to one of its physiological ligands that results in the spatial identity of regions along the anterior-posterior axis of the spinal cord.